{
  "gene": "UniProtKB:Q6ZVT6",
  "term_id": "UNKNOWN:0002",
  "gene_name": "Protein CFAP20DC",
  "gene_symbol": "CFAP20DC",
  "term_label": "Unknown biological process"
}